low-affinity phosphate transmembrane transporter activity [GO:0009673] (molecular function) Sources: TC:2.A.20.-.- Definition: Enables the transfer of phosphate from one side of a membrane to the other. In low-affinity transport the transporter is able to bind the solute only if it is present at very high concentrations. Relationships: is a type of phosphate transmembrane transporter activity [GO:0005315] Also known as: low affinity phosphate transmembrane transporter activity